{
  "gene_symbol": "VENTX",
  "gene": "UniProtKB:O95231",
  "gene_name": "Homeobox protein VENTX",
  "term_label": "DNA-binding transcription factor activity, RNA polymerase II-specific",
  "term_id": "GO:0000981"
}